regulation of positive chemotaxis to cAMP [GO:0061118] (biological process) Definition: Any process that modulates the rate, frequency, or extent of directed movement of a motile cell or organism up a concentration gradient of 3',5'-cAMP. Subtypes: GO:0061119, positive regulation of positive chemotaxis to cAMP [GO:0061122], negative regulation of positive chemotaxis to cAMP [GO:0061123] Sources: GOC:dph Relationships: is a type of regulation of positive chemotaxis [GO:0050926]; regulates chemotaxis to cAMP [GO:0043327]